{
  "term_label": "GTPase activator activity",
  "gene_name": "Arf-GAP with GTPase, ANK repeat and PH domain-containing protein 9",
  "term_id": "GO:0005096",
  "gene": "UniProtKB:Q5VTM2",
  "gene_symbol": "AGAP9"
}